integrin alpha9-beta1 complex [GO:0034679] (cellular component) Relationships: is a type of GO:0008305 Also known as: alpha9-beta1 integrin complex, ITGA9-ITGB1 complex Definition: An integrin complex that comprises one alpha9 subunit and one beta1 subunit. References: PMID:12297042